{
  "gene_name": "WW domain-containing oxidoreductase",
  "gene_symbol": "WWOX",
  "gene": "UniProtKB:Q9NZC7",
  "term_id": "UNKNOWN:0002",
  "term_label": "Unknown biological process"
}